{
  "gene": "UniProtKB:Q96P65",
  "term_id": "GO:0004930",
  "gene_name": "Pyroglutamylated RF-amide peptide receptor",
  "gene_symbol": "QRFPR",
  "term_label": "G protein-coupled receptor activity"
}